septum digestion after cytokinesis [GO:0000920] (biological process) Note: This term should not be used to describe the last step of cytokinesis in organisms without a cell wall, ie, the cell resealing of the plasma membrane via abscission. Consider annotating to 'GO:0061952 midbody abscission' to capture this process. Sources: GOC:mtg_cell_cycle, GOC:vw Definition: The process of physically separating the septal cell wall material by enzymatic digestion, that occurs after daughter cells are separated by cytokinesis. Regulation: regulated by regulation of septum digestion after cytokinesis [GO:0010590]; negatively regulated by negative regulation of septum digestion after cytokinesis [GO:2001042]; positively regulated by positive regulation of septum digestion after cytokinesis [GO:2001043] Relationships: is a type of GO:0009987; is part of GO:0051301 Also known as: mitotic cytokinetic cell separation, cell separation following cytokinesis, cell separation after cytokinesis, cytokinetic cell separation, daughter cell separation